glyceraldehyde-3-phosphate dehydrogenase (NADP+) (non-phosphorylating) activity [GO:0008886] (MF) Relationships: is a type of glyceraldehyde-3-phosphate dehydrogenase [NAD(P)+] (non-phosphorylating) activity [GO:0120533] Also known as: NADP-glyceraldehyde phosphate dehydrogenase, dehydrogenase, glyceraldehyde phosphate (nicotinamide adenine dinucleotide phosphate), glyceraldehyde phosphate dehydrogenase (NADP), triosephosphate dehydrogenase activity, D-glyceraldehyde-3-phosphate:NADP+ oxidoreductase activity, NADP-glyceraldehyde-3-phosphate dehydrogenase activity, glyceraldehyde 3-phosphate dehydrogenase (NADP), glyceraldehyde-3-phosphate dehydrogenase (NADP), glyceraldehyde-3-phosphate:NADP reductase activity, nonphosphorylating glyceraldehyde-3-phosphate dehydrogenase activity Definition: Catalysis of the reaction: D-glyceraldehyde 3-phosphate + H2O + NADP+ = 3-phospho-D-glycerate + 2 H+ + NADPH. Sources: EC:1.2.1.9, RHEA:14669